phosphatidylinositol N-acetylglucosaminyltransferase activity [GO:0017176] (molecular function) Definition: Catalysis of the reaction: UDP-N-acetyl-D-glucosamine + phosphatidylinositol = UDP + N-acetyl-D-glucosaminylphosphatidylinositol. Also known as: UDP-N-acetyl-D-glucosamine:1-phosphatidyl-1D-myo-inositol 6-(N-acetyl-alpha-D-glucosaminyl)transferase activity, UDP-N-acetyl-D-glucosamine:phosphatidylinositol N-acetyl-D-glucosaminyltransferase activity, uridine diphosphoacetylglucosamine alpha-1,6-acetyl-D-glucosaminyltransferase activity, uridine diphosphoacetylglucosamine alpha1,6-acetyl-D-glucosaminyltransferase activity Relationships: is_a acetylglucosaminyltransferase activity [GO:0008375] Sources: EC:2.4.1.198